{
  "gene_name": "Probable non-functional immunoglobulin kappa variable 3-7",
  "term_label": "immunoglobulin complex",
  "term_id": "GO:0019814",
  "gene_symbol": "IGKV3-7",
  "gene": "UniProtKB:A0A075B6H7"
}